{
  "gene": "UniProtKB:Q96SN8",
  "term_label": "microtubule bundle formation",
  "gene_name": "CDK5 regulatory subunit-associated protein 2",
  "term_id": "GO:0001578",
  "gene_symbol": "CDK5RAP2"
}